regulation of protein localization to membrane [GO:1905475] (BP) References: PMID:26911690 Sources: GOC:PARL, GOC:TermGenie, GOC:bc, GO_REF:0000058 Relationships: is a type of regulation of protein localization [GO:0032880]; is a type of GO:0060341; RO_0002211 protein localization to membrane [GO:0072657] Subtypes: regulation of neurotransmitter receptor localization to postsynaptic specialization membrane [GO:0098696], GO:0099145, regulation of protein targeting to vacuolar membrane [GO:1900483], regulation of postsynaptic density protein 95 clustering [GO:1902897], regulation of protein localization to plasma membrane [GO:1903076], GO:1903567, regulation of receptor clustering [GO:1903909], regulation of t-SNARE clustering [GO:1904032], regulation of protein localization to basolateral plasma membrane [GO:1904508], negative regulation of protein localization to membrane [GO:1905476], positive regulation of protein localization to membrane [GO:1905477] Also known as: regulation of protein localisation in membrane, regulation of protein localization in membrane Definition: Any process that modulates the frequency, rate or extent of protein localization to membrane.